{
  "gene_symbol": "KNCN",
  "term_id": "GO:0060091",
  "gene_name": "Kinocilin",
  "gene": "UniProtKB:A6PVL3",
  "term_label": "kinocilium"
}